{
  "gene_name": "Anaphase-promoting complex subunit 15",
  "gene_symbol": "ANAPC15",
  "term_id": "UNKNOWN:0001",
  "gene": "UniProtKB:P60006",
  "term_label": "Unknown molecular function"
}